{
  "gene_symbol": "PEMT",
  "gene": "UniProtKB:Q9UBM1",
  "term_id": "UNKNOWN:0003",
  "term_label": "Unknown cellular component",
  "gene_name": "Phosphatidylethanolamine N-methyltransferase"
}